regulation of secretion by cell [GO:1903530] (biological process) Definition: Any process that modulates the frequency, rate or extent of secretion by cell. References: PMID:12130530 Sources: GOC:TermGenie, GOC:pm, GO_REF:0000058 Also known as: regulation of cellular secretion Relationships: is a type of regulation of cellular process [GO:0050794]; is a type of GO:0051046; regulates GO:0032940 Subtypes: regulation of extracellular matrix constituent secretion [GO:0003330], regulation of glutamate secretion [GO:0014048], regulation of serotonin secretion [GO:0014062], regulation of exocytosis [GO:0017157], regulation of prostaglandin secretion [GO:0032306], GO:0046883, GO:0046928, regulation of catecholamine secretion [GO:0050433], regulation of protein secretion [GO:0050708], GO:1903531, positive regulation of secretion by cell [GO:1903532], GO:1904448